{
  "term_label": "nucleus",
  "gene_symbol": "FGF13",
  "gene_name": "Fibroblast growth factor 13",
  "term_id": "GO:0005634",
  "gene": "UniProtKB:Q92913"
}